{
  "gene": "UniProtKB:Q9BYQ5",
  "term_id": "UNKNOWN:0001",
  "gene_name": "Keratin-associated protein 4-6",
  "gene_symbol": "KRTAP4-6",
  "term_label": "Unknown molecular function"
}